{
  "gene_name": "C-C motif chemokine 15",
  "gene_symbol": "CCL15",
  "term_id": "GO:0048020",
  "gene": "UniProtKB:Q16663",
  "term_label": "CCR chemokine receptor binding"
}